{
  "term_id": "GO:0006887",
  "gene_symbol": "STX11",
  "term_label": "exocytosis",
  "gene_name": "Syntaxin-11",
  "gene": "UniProtKB:O75558"
}